{
  "gene_symbol": "SHQ1",
  "gene_name": "Protein SHQ1 homolog",
  "term_label": "unfolded protein binding",
  "gene": "UniProtKB:Q6PI26",
  "term_id": "GO:0051082"
}